{
  "term_id": "GO:0005794",
  "gene_symbol": "SYAP1",
  "gene_name": "Synapse-associated protein 1",
  "gene": "UniProtKB:Q96A49",
  "term_label": "Golgi apparatus"
}